{
  "gene_name": "BTB_POZ domain-containing protein KCTD12",
  "gene": "UniProtKB:Q96CX2",
  "term_id": "UNKNOWN:0001",
  "term_label": "Unknown molecular function",
  "gene_symbol": "KCTD12"
}